{
  "gene_name": "Mitochondrial import receptor subunit TOM40 homolog",
  "term_label": "protein transmembrane transporter activity",
  "gene_symbol": "TOMM40",
  "term_id": "GO:0008320",
  "gene": "UniProtKB:O96008"
}